octopamine signaling pathway involved in response to food [GO:0071935] (biological process) Relationships: is a type of octopamine signaling pathway [GO:0071927]; is part of response to food [GO:0032094] Regulation: regulated by regulation of octopamine signaling pathway involved in response to food [GO:2000139]; negatively regulated by negative regulation of octopamine signaling pathway involved in response to food [GO:2000140]; positively regulated by positive regulation of octopamine signaling pathway involved in response to food [GO:2000141] References: PMID:19609300 Sources: GOC:mah Also known as: octopamine signalling pathway involved in response to food Definition: The series of molecular signals initiated by binding of octopamine to a receptor on the surface of the target cell that contributes to a response to a food stimulus.